regulation of AV node cell action potential [GO:0098904] (biological process) Relationships: is a type of regulation of cell communication [GO:0010646]; is a type of GO:0098901; regulates GO:0086016 Subtypes: GO:1903950, positive regulation of AV node cell action potential [GO:1903951], regulation of membrane depolarization during AV node cell action potential [GO:1905027] Sources: GOC:BHF, GOC:mtg_cardiac_conduct_nov11 Definition: Any process that modulates the frequency, rate or extent of action potential creation, propagation or termination in an atrioventricular node myocyte. This typically occurs via modulation of the activity or expression of voltage-gated ion channels. Also known as: regulation of AV node cardiac muscle cell action potential, regulation of atrioventricular node cardiac muscle cell action potential